peptidyl-histidine modification [GO:0018202] (biological process) Subtypes: protein histidyl modification to diphthamide [GO:0017183], peptidyl-histidine methylation [GO:0018021], peptidyl-histidine phosphorylation [GO:0018106], nickel incorporation into iron-sulfur cluster via tris-L-cysteinyl L-cysteine persulfido L-glutamato L-histidino L-serinyl nickel triiron disulfide trioxide [GO:0018418], peptidyl-histidine adenylylation [GO:0051111], peptidyl-histidine uridylylation [GO:0051114] Relationships: is a type of GO:0018193 Definition: The modification of peptidyl-histidine. Sources: GOC:ma